{
  "gene": "UniProtKB:Q10471",
  "term_id": "GO:0006493",
  "gene_symbol": "GALNT2",
  "gene_name": "Polypeptide N-acetylgalactosaminyltransferase 2",
  "term_label": "protein O-linked glycosylation"
}